{
  "gene_symbol": "SARNP",
  "gene_name": "SAP domain-containing ribonucleoprotein",
  "term_id": "GO:0005634",
  "term_label": "nucleus",
  "gene": "UniProtKB:P82979"
}